{
  "gene_name": "Pregnancy-specific beta-1-glycoprotein 4",
  "term_id": "UNKNOWN:0001",
  "term_label": "Unknown molecular function",
  "gene": "UniProtKB:Q00888",
  "gene_symbol": "PSG4"
}